{
  "gene_symbol": "RNASE2",
  "gene_name": "Non-secretory ribonuclease",
  "term_label": "chemotaxis",
  "term_id": "GO:0006935",
  "gene": "UniProtKB:P10153"
}